{
  "term_id": "GO:0035023",
  "gene": "UniProtKB:Q96BY6",
  "gene_name": "Dedicator of cytokinesis protein 10",
  "term_label": "regulation of Rho protein signal transduction",
  "gene_symbol": "DOCK10"
}